positive regulation of lipoprotein metabolic process [GO:0050747] (biological process) Also known as: positive regulation of lipoprotein metabolism, up regulation of lipoprotein metabolic process, up-regulation of lipoprotein metabolic process, upregulation of lipoprotein metabolic process, activation of lipoprotein metabolic process, stimulation of lipoprotein metabolic process Definition: Any process that activates or increases the frequency, rate or extent of the chemical reactions and pathways involving lipoproteins, any conjugated, water-soluble protein in which the nonprotein group consists of a lipid or lipids. Sources: GOC:ai Relationships: is a type of positive regulation of biosynthetic process [GO:0009891]; is a type of GO:0050746; is a type of positive regulation of protein metabolic process [GO:0051247]; positively regulates lipoprotein metabolic process [GO:0042157] Subtypes: GO:1903061